{
  "gene_symbol": "AQP7",
  "gene_name": "Aquaporin-7",
  "gene": "UniProtKB:O14520",
  "term_id": "GO:0015250",
  "term_label": "water channel activity"
}